{
  "gene_symbol": "RAD9A",
  "term_label": "mitotic intra-S DNA damage checkpoint signaling",
  "gene_name": "Cell cycle checkpoint control protein RAD9A",
  "term_id": "GO:0031573",
  "gene": "UniProtKB:Q99638"
}